{
  "gene_name": "Poly [ADP-ribose] polymerase 2",
  "gene": "UniProtKB:Q9UGN5",
  "term_id": "GO:0006302",
  "term_label": "double-strand break repair",
  "gene_symbol": "PARP2"
}